{
  "gene_name": "Small cysteine and glycine repeat-containing protein 2",
  "term_id": "UNKNOWN:0002",
  "gene": "UniProtKB:A0A286YFB4",
  "gene_symbol": "SCYGR2",
  "term_label": "Unknown biological process"
}